{
  "gene_symbol": "CDH13",
  "gene": "UniProtKB:P55290",
  "gene_name": "Cadherin-13",
  "term_id": "GO:0016339",
  "term_label": "calcium-dependent cell-cell adhesion"
}